{
  "gene_symbol": "ADI1",
  "term_label": "acireductone dioxygenase [iron(II)-requiring] activity",
  "term_id": "GO:0010309",
  "gene_name": "Acireductone dioxygenase",
  "gene": "UniProtKB:Q9BV57"
}